positive regulation of angiotensin-activated signaling pathway [GO:0110063] (biological process) Relationships: is a type of GO:0045745; is a type of GO:0110061; positively regulates angiotensin-activated signaling pathway [GO:0038166] References: PMID:28784619 Sources: GOC:lf Definition: Any process that activates or increases the frequency, rate or extent of the angiotensin-activated signaling pathway.